{
  "term_id": "UNKNOWN:0003",
  "gene_name": "DENN domain-containing protein 2C",
  "gene_symbol": "DENND2C",
  "gene": "UniProtKB:Q68D51",
  "term_label": "Unknown cellular component"
}